{
  "gene_symbol": "CHP2",
  "term_id": "GO:0005509",
  "gene": "UniProtKB:O43745",
  "gene_name": "Calcineurin B homologous protein 2",
  "term_label": "calcium ion binding"
}